{
  "gene_symbol": "CMKLR2",
  "gene": "UniProtKB:P46091",
  "gene_name": "Chemerin-like receptor 2",
  "term_id": "GO:0042923",
  "term_label": "neuropeptide binding"
}